U2-type prespliceosome [GO:0071004] (cellular component) Definition: A spliceosomal complex that is formed by association of the 5' splice site with the U1 snRNP, while the branch point sequence is recognized by the U2 snRNP. The prespliceosome includes many proteins in addition to those found in the U1 and U2 snRNPs. Commitment to a given pair of 5' and 3' splice sites occurs at the time of prespliceosome formation. Relationships: is a type of GO:0005684; is_a prespliceosome [GO:0071010]; has part U1 snRNP [GO:0005685]; has part GO:0005686 Also known as: major prespliceosome, GT-AG prespliceosome, mammalian U2-type spliceosomal complex A, yeast U2-type spliceosomal complex B References: PMID:17332742, PMID:19239890 Sources: GOC:ab, GOC:krc, GOC:mah